energy transducer activity [GO:0031992] (molecular function) Also known as: light harvesting activity, photon capture Sources: GOC:go_curators Definition: The biological transducer activity that accepts energy and converts it to another form, often by transfer to another molecule within the cell. Subtypes: light transducer activity [GO:0031993] Relationships: is a type of molecular transducer activity [GO:0060089]